{
  "gene_name": "CXADR-like membrane protein",
  "gene": "UniProtKB:Q9H6B4",
  "term_label": "Unknown molecular function",
  "term_id": "UNKNOWN:0001",
  "gene_symbol": "CLMP"
}